toluene dioxygenase activity [GO:0018624] (molecular function) Sources: EC:1.14.12.11, RHEA:16737 Definition: Catalysis of the reaction: H+ + NADH + O2 + toluene = (1S,2R)-3-methylcyclohexa-3,5-diene-1,2-diol + NAD+. Relationships: is a type of oxidoreductase activity, acting on paired donors, with incorporation or reduction of molecular oxygen, NAD(P)H as one donor, and incorporation of two atoms of oxygen into one donor [GO:0016708] Also known as: toluene 1,2-dioxygenase activity, toluene 2,3-dioxygenase activity, toluene,NADH:oxygen oxidoreductase (1,2-hydroxylating)